{
  "term_label": "synaptic vesicle membrane",
  "gene_symbol": "FER1L5",
  "gene": "UniProtKB:A0AVI2",
  "gene_name": "Fer-1-like protein 5",
  "term_id": "GO:0030672"
}